response to molybdenum starvation [GO:0090550] (biological process) Relationships: is a type of GO:0042594 Definition: Any process that results in a change in state or activity of a cell or an organism (in terms of movement, secretion, enzyme production, gene expression, etc.) as a result of a starvation stimulus, deprivation of molybdenum. Sources: GOC:tair_curators